{
  "gene_name": "RB1-inducible coiled-coil protein 1",
  "term_id": "GO:0000425",
  "gene": "UniProtKB:Q8TDY2",
  "term_label": "pexophagy",
  "gene_symbol": "RB1CC1"
}